{
  "term_label": "ubiquitin conjugating enzyme activity",
  "gene_name": "Ubiquitin-conjugating enzyme E2 Q1",
  "gene_symbol": "UBE2Q1",
  "gene": "UniProtKB:Q7Z7E8",
  "term_id": "GO:0061631"
}